{
  "gene": "UniProtKB:Q9NXR7",
  "term_label": "BRCA1-A complex",
  "gene_name": "BRISC and BRCA1-A complex member 2",
  "gene_symbol": "BABAM2",
  "term_id": "GO:0070531"
}